{
  "gene": "UniProtKB:P42262",
  "gene_name": "Glutamate receptor 2",
  "gene_symbol": "GRIA2",
  "term_id": "GO:0004971",
  "term_label": "AMPA glutamate receptor activity"
}